storage vacuole [GO:0000322] (cellular component) Sources: GOC:krc Definition: A vacuole that functions primarily in the storage of materials, including nutrients, pigments, waste products, and small molecules. Subtypes: fungal-type vacuole [GO:0000324], protein storage vacuole [GO:0000326], reservosome [GO:0106123] Relationships: is a type of vacuole [GO:0005773]